{
  "gene": "UniProtKB:Q9Y291",
  "gene_symbol": "MRPS33",
  "gene_name": "Small ribosomal subunit protein mS33",
  "term_label": "Unknown biological process",
  "term_id": "UNKNOWN:0002"
}